{
  "term_id": "GO:0015459",
  "term_label": "potassium channel regulator activity",
  "gene": "UniProtKB:Q9NS61",
  "gene_symbol": "KCNIP2",
  "gene_name": "Kv channel-interacting protein 2"
}